regulation of interphase mitotic telomere clustering [GO:0110065] (biological process) References: PMID:25778919 Sources: GOC:vw Definition: Any process that modulates the frequency, rate or extent of mitotic telomere clustering during interphase. Relationships: is a type of regulation of localization [GO:0032879]; regulates interphase mitotic telomere clustering [GO:0120110] Subtypes: GO:0110066 Also known as: regulation of mitotic telomere clustering during interphase